{
  "gene_name": "Zinc finger protein 7",
  "term_id": "GO:0005634",
  "gene_symbol": "ZNF7",
  "term_label": "nucleus",
  "gene": "UniProtKB:P17097"
}